regulation of smooth muscle cell differentiation [GO:0051150] (biological process) Definition: Any process that modulates the frequency, rate or extent of smooth muscle cell differentiation. Relationships: is a type of regulation of muscle cell differentiation [GO:0051147]; regulates GO:0051145 Subtypes: negative regulation of smooth muscle cell differentiation [GO:0051151], positive regulation of smooth muscle cell differentiation [GO:0051152], GO:1905063, regulation of ureter smooth muscle cell differentiation [GO:2000061], regulation of kidney smooth muscle cell differentiation [GO:2000356] Sources: CL:0000192, GOC:ai